anaerobic glycerol catabolic process to propane-1,3-diol [GO:0019589] (biological process) Also known as: glycerol fermentation to 1,3-propanediol, glycerol fermentation to propane-1,3-diol Definition: The anaerobic chemical reactions and pathways resulting in the breakdown of glycerol into propane-1,3-diol and water. Sources: GOC:jl, MetaCyc:GOLPDLCAT-PWY Relationships: is a type of anaerobic glycerol catabolic process [GO:0019588]; is a type of GO:0042844